{
  "gene_symbol": "LGALS2",
  "gene_name": "Galectin-2",
  "term_id": "GO:0016936",
  "gene": "UniProtKB:P05162",
  "term_label": "galactoside binding"
}